{
  "term_label": "kinetochore assembly",
  "term_id": "GO:0051382",
  "gene_symbol": "CENPA",
  "gene_name": "Histone H3-like centromeric protein A",
  "gene": "UniProtKB:P49450"
}